{
  "gene": "UniProtKB:A0A0B4J280",
  "term_id": "GO:0019814",
  "gene_name": "T cell receptor alpha variable 40",
  "gene_symbol": "TRAV40",
  "term_label": "immunoglobulin complex"
}